toluene oxidation via 4-hydroxytoluene [GO:0019603] (biological process) Relationships: is a type of toluene oxidation [GO:0019600] Definition: The degradation of toluene to form p-hydroxybenzoate; the first step in the pathway is the oxidation of toluene to form 4-hydroxytoluene (4-cresol). Sources: MetaCyc:TOLUENE-DEG-4-OH-PWY